response to antimetabolite [GO:0097329] (biological process) Definition: Any process that results in a change in state or activity of a cell or an organism (in terms of movement, secretion, enzyme production, gene expression, etc.) as a result of an antimetabolite stimulus. An antimetabolite is a substance which is structurally similar to a metabolite but which competes with it or replaces it, and so prevents or reduces its normal utilization. Sources: GOC:pr Relationships: is_a response to chemical [GO:0042221]